{
  "gene_symbol": "SSH2",
  "term_id": "GO:0004721",
  "gene_name": "Protein phosphatase Slingshot homolog 2",
  "term_label": "phosphoprotein phosphatase activity",
  "gene": "UniProtKB:Q76I76"
}